virion component [GO:0044423] (cellular component) Relationships: is a type of GO:0005575 Subtypes: GO:0019013, viral capsid [GO:0019028], viral tegument [GO:0019033], viral membrane [GO:0036338], viral outer capsid [GO:0039624], viral inner capsid [GO:0039625], GO:0039626, virion nucleoid [GO:0039642], capsomere [GO:0046727], GO:0046729, GO:0055036, GO:0098015, viral capsid, decoration [GO:0098021], virus tail, tip [GO:0098023], virus tail, fiber [GO:0098024], GO:0098025, GO:0098026, GO:0098027, virus tail, shaft [GO:0098028], GO:0098029, icosahedral viral capsid, neck [GO:0098030], icosahedral viral capsid, collar [GO:0098031], GO:0098061 Also known as: virion part, complete virus particle, virion Sources: GOC:jl Definition: Any constituent part of a virion, a complete fully infectious extracellular virus particle.